methylglyoxal reductase (NADPH) (acetol producing) activity [GO:1990002] (molecular function) References: PMID:16077126 Sources: RHEA:27986 Definition: Catalysis of the reaction: hydroxyacetone + NADP+ = H+ + methylglyoxal + NADPH. Relationships: is a type of oxidoreductase activity, acting on the CH-OH group of donors, NAD or NADP as acceptor [GO:0016616] Also known as: methylglyoxal reductase (NADPH-dependent, acetol producing)